{
  "gene_symbol": "ANXA9",
  "gene": "UniProtKB:O76027",
  "term_label": "cytoplasm",
  "term_id": "GO:0005737",
  "gene_name": "Annexin A9"
}